{
  "gene_name": "Transcription factor HES-7",
  "term_id": "GO:0050767",
  "term_label": "regulation of neurogenesis",
  "gene": "UniProtKB:Q9BYE0",
  "gene_symbol": "HES7"
}